neutrophil-mediated killing of bacterium [GO:0070944] (biological process) Relationships: is a type of neutrophil-mediated killing of symbiont cell [GO:0070943]; is part of defense response to bacterium [GO:0042742] Also known as: neutrophil mediated killing of bacterium Sources: GOC:add, ISBN:0781765196 Definition: The directed killing of a bacterium by a neutrophil. Subtypes: neutrophil-mediated killing of gram-negative bacterium [GO:0070945], GO:0070946 Regulation: regulated by regulation of neutrophil mediated killing of bacterium [GO:0070950]; negatively regulated by GO:0070956; positively regulated by positive regulation of neutrophil mediated killing of bacterium [GO:0070962]